{
  "gene_name": "Epidermal growth factor receptor kinase substrate 8-like protein 2",
  "term_id": "GO:0003779",
  "gene_symbol": "EPS8L2",
  "term_label": "actin binding",
  "gene": "UniProtKB:Q9H6S3"
}